negative regulation of otic vesicle morphogenesis [GO:1904119] (biological process) Definition: Any process that stops, prevents or reduces the frequency, rate or extent of otic vesicle morphogenesis. References: PMID:25677106 Sources: GOC:TermGenie, GO_REF:0000058 Relationships: is a type of negative regulation of animal organ morphogenesis [GO:0110111]; is a type of regulation of otic vesicle morphogenesis [GO:1904118]; is a type of negative regulation of morphogenesis of an epithelium [GO:1905331]; RO_0002212 otic vesicle morphogenesis [GO:0071600] Also known as: down regulation of otic vesicle morphogenesis, down-regulation of otic vesicle morphogenesis, downregulation of otic vesicle morphogenesis, inhibition of otic vesicle morphogenesis